{
  "gene_symbol": "SALL4",
  "term_id": "GO:0006357",
  "term_label": "regulation of transcription by RNA polymerase II",
  "gene": "UniProtKB:Q9UJQ4",
  "gene_name": "Sal-like protein 4"
}